{
  "gene_name": "Protein 4.1",
  "gene_symbol": "EPB41",
  "term_label": "plasma membrane",
  "term_id": "GO:0005886",
  "gene": "UniProtKB:P11171"
}